{
  "term_label": "metalloaminopeptidase activity",
  "term_id": "GO:0070006",
  "gene_name": "Aminopeptidase B",
  "gene_symbol": "RNPEP",
  "gene": "UniProtKB:Q9H4A4"
}